{
  "gene": "UniProtKB:P17483",
  "term_label": "nucleoplasm",
  "term_id": "GO:0005654",
  "gene_symbol": "HOXB4",
  "gene_name": "Homeobox protein Hox-B4"
}